{
  "gene": "UniProtKB:Q9H171",
  "term_label": "positive regulation of type I interferon-mediated signaling pathway",
  "gene_symbol": "ZBP1",
  "term_id": "GO:0060340",
  "gene_name": "Z-DNA-binding protein 1"
}